{
  "gene": "UniProtKB:Q13536",
  "gene_symbol": "MIR9-1HG",
  "gene_name": "Protein CROC-4",
  "term_label": "Unknown molecular function",
  "term_id": "UNKNOWN:0001"
}